{
  "term_label": "structural constituent of ribosome",
  "gene_name": "Large ribosomal subunit protein uL24m",
  "gene_symbol": "MRPL24",
  "term_id": "GO:0003735",
  "gene": "UniProtKB:Q96A35"
}